{
  "gene": "UniProtKB:Q02817",
  "gene_name": "Mucin-2",
  "term_id": "UNKNOWN:0003",
  "gene_symbol": "MUC2",
  "term_label": "Unknown cellular component"
}